{
  "gene": "UniProtKB:Q9Y5L4",
  "term_label": "Unknown molecular function",
  "gene_symbol": "TIMM13",
  "term_id": "UNKNOWN:0001",
  "gene_name": "Mitochondrial import inner membrane translocase subunit Tim13"
}